disaccharide metabolic process [GO:0005984] (biological process) Relationships: is a type of GO:0009311 Also known as: disaccharide metabolism Sources: GOC:jl, ISBN:0192800981 Subtypes: GO:0000023, GO:0005985, lactose metabolic process [GO:0005988], trehalose metabolic process [GO:0005991], disaccharide biosynthetic process [GO:0046351], disaccharide catabolic process [GO:0046352], cellobiose metabolic process [GO:2000891] Definition: The chemical reactions and pathways involving any disaccharide, sugars composed of two monosaccharide units.